{
  "term_label": "Unknown molecular function",
  "term_id": "UNKNOWN:0001",
  "gene": "UniProtKB:Q9P209",
  "gene_symbol": "CEP72",
  "gene_name": "Centrosomal protein of 72 kDa"
}